{
  "term_label": "Unknown cellular component",
  "gene_symbol": "ADAM12",
  "gene_name": "Disintegrin and metalloproteinase domain-containing protein 12",
  "term_id": "UNKNOWN:0003",
  "gene": "UniProtKB:O43184"
}